{
  "gene_name": "Caspase-8",
  "gene_symbol": "CASP8",
  "term_label": "macrophage differentiation",
  "term_id": "GO:0030225",
  "gene": "UniProtKB:Q14790"
}